C zone [GO:0014705] (cellular component) Sources: GOC:mtg_muscle Relationships: is a type of GO:0110165; is part of GO:0031672 Definition: A region of the A band in which myosin-binding protein C is located and that can be seen by electron microscopy. This is a functional zone that also includes myosin.